{
  "gene": "UniProtKB:Q8N6D2",
  "gene_name": "E3 ubiquitin-protein ligase RNF182",
  "gene_symbol": "RNF182",
  "term_id": "GO:0016567",
  "term_label": "protein ubiquitination"
}